{
  "gene_name": "Zinc-regulated GTPase metalloprotein activator 1C",
  "gene_symbol": "ZNG1C",
  "term_id": "GO:0051604",
  "term_label": "protein maturation",
  "gene": "UniProtKB:Q5JTY5"
}